laminin-6 complex [GO:0005611] (cellular component) Relationships: is a type of GO:0043256 References: PMID:10842354 Sources: GOC:jl Also known as: laminin-311 complex, laminin-6A complex Definition: A laminin complex composed of alpha3, beta1 and gamma1 polypeptide chains.